{
  "gene": "UniProtKB:Q8N138",
  "gene_name": "ORM1-like protein 3",
  "term_id": "GO:0030148",
  "gene_symbol": "ORMDL3",
  "term_label": "sphingolipid biosynthetic process"
}